{
  "term_id": "GO:0005634",
  "term_label": "nucleus",
  "gene_name": "Condensin-2 complex subunit G2",
  "gene_symbol": "NCAPG2",
  "gene": "UniProtKB:Q86XI2"
}